{
  "gene": "UniProtKB:A0A075B6I9",
  "gene_name": "Immunoglobulin lambda variable 7-46",
  "term_id": "UNKNOWN:0001",
  "gene_symbol": "IGLV7-46",
  "term_label": "Unknown molecular function"
}